{
  "term_label": "Unknown molecular function",
  "gene_symbol": "THBS2",
  "term_id": "UNKNOWN:0001",
  "gene_name": "Thrombospondin-2",
  "gene": "UniProtKB:P35442"
}